macrophage colony-stimulating factor signaling pathway [GO:0038145] (biological process) Definition: The series of molecular signals initiated by the binding of the cytokine macrophage colony-stimulating factor (M-CSF) to its receptor on the surface of a target cell, and ending with the regulation of a downstream cellular process, e.g. transcription. References: PMID:12138890 Sources: GOC:signaling, GOC:uh, Wikipedia:Macrophage_colony-stimulating_factor Also known as: M-CSF signaling pathway, macrophage colony-stimulating factor signalling pathway Relationships: is a type of cytokine-mediated signaling pathway [GO:0019221]; is part of cellular response to macrophage colony-stimulating factor stimulus [GO:0036006] Regulation: regulated by regulation of macrophage colony-stimulating factor signaling pathway [GO:1902226]; negatively regulated by negative regulation of macrophage colony-stimulating factor signaling pathway [GO:1902227]; positively regulated by positive regulation of macrophage colony-stimulating factor signaling pathway [GO:1902228]